{
  "term_label": "Unknown molecular function",
  "gene_name": "Sec1 family domain-containing protein 2",
  "gene_symbol": "SCFD2",
  "term_id": "UNKNOWN:0001",
  "gene": "UniProtKB:Q8WU76"
}